{
  "gene": "UniProtKB:Q9NRV9",
  "term_id": "UNKNOWN:0003",
  "term_label": "Unknown cellular component",
  "gene_symbol": "HEBP1",
  "gene_name": "Heme-binding protein 1"
}